glycogen catabolic process [GO:0005980] (biological process) Definition: The chemical reactions and pathways resulting in the breakdown of glycogen, a polydisperse, highly branched glucan composed of chains of D-glucose residues. Subtypes: GO:0061723, glycogen catabolic process via dextrin [GO:0160251], GO:0160252 Regulation: regulated by regulation of glycogen catabolic process [GO:0005981]; negatively regulated by negative regulation of glycogen catabolic process [GO:0045818]; positively regulated by positive regulation of glycogen catabolic process [GO:0045819] Relationships: is a type of GO:0005977; is a type of glucan catabolic process [GO:0009251] Also known as: glycogen breakdown, glycogen catabolism, glycogen degradation, glycogenolysis Sources: ISBN:0198506732